{
  "gene_symbol": "TIGD7",
  "term_label": "Unknown biological process",
  "gene_name": "Tigger transposable element-derived protein 7",
  "term_id": "UNKNOWN:0002",
  "gene": "UniProtKB:Q6NT04"
}